{
  "gene_symbol": "ACSM5",
  "gene": "UniProtKB:Q6NUN0",
  "term_id": "GO:0004321",
  "term_label": "fatty-acyl-CoA synthase activity",
  "gene_name": "Acyl-coenzyme A synthetase ACSM5, mitochondrial"
}